negative regulation of syncytium formation by plasma membrane fusion [GO:0034242] (biological process) Relationships: is a type of negative regulation of developmental process [GO:0051093]; is a type of negative regulation of cellular component organization [GO:0051129]; is_a regulation of syncytium formation by plasma membrane fusion [GO:0060142]; negatively regulates syncytium formation by plasma membrane fusion [GO:0000768] Subtypes: negative regulation of macrophage fusion [GO:0034240], negative regulation of myoblast fusion [GO:1901740] Sources: GOC:mah Definition: Any process that decreases the frequency, rate or extent of the formation of a syncytium, a mass of cytoplasm containing several nuclei enclosed within a single plasma membrane, by the fusion of the plasma membranes of two or more individual cells.